{
  "gene_name": "Colipase",
  "gene": "UniProtKB:P04118",
  "term_id": "GO:0008047",
  "term_label": "enzyme activator activity",
  "gene_symbol": "CLPS"
}